{
  "term_label": "rRNA processing",
  "gene": "UniProtKB:Q99848",
  "term_id": "GO:0006364",
  "gene_symbol": "EBNA1BP2",
  "gene_name": "Probable rRNA-processing protein EBP2"
}